{
  "gene_name": "Equatorin",
  "gene_symbol": "EQTN",
  "gene": "UniProtKB:Q9NQ60",
  "term_label": "acrosomal vesicle exocytosis",
  "term_id": "GO:0060478"
}